{
  "gene_name": "Vasopressin V1b receptor",
  "gene": "UniProtKB:P47901",
  "gene_symbol": "AVPR1B",
  "term_id": "GO:0005000",
  "term_label": "vasopressin receptor activity"
}